{
  "gene_name": "AP-3 complex subunit mu-1",
  "term_label": "AP-1 adaptor complex",
  "gene_symbol": "AP3M1",
  "gene": "UniProtKB:Q9Y2T2",
  "term_id": "GO:0030121"
}